{
  "term_label": "enzyme-substrate adaptor activity",
  "term_id": "GO:0140767",
  "gene_name": "Cell division cycle protein 27 homolog",
  "gene_symbol": "CDC27",
  "gene": "UniProtKB:P30260"
}